{
  "gene_symbol": "ING5",
  "gene": "UniProtKB:Q8WYH8",
  "gene_name": "Inhibitor of growth protein 5",
  "term_label": "nucleus",
  "term_id": "GO:0005634"
}